peptidyl-histidine methylation, to form tele-methylhistidine [GO:0042038] (biological process) Sources: RESID:AA0317 Also known as: peptidyl-histidine tele-methylation Relationships: is a type of peptidyl-histidine methylation [GO:0018021] Definition: The methylation of peptidyl-L-histidine to form peptidyl-L-1'-methyl-L-histidine (otherwise known as tau-methylhistidine, tele-methylhistidine).